{
  "gene": "UniProtKB:Q8TAM6",
  "term_label": "morphogenesis of a branching structure",
  "term_id": "GO:0001763",
  "gene_symbol": "ERMN",
  "gene_name": "Ermin"
}